{
  "gene_name": "Transmembrane 9 superfamily member 3",
  "gene_symbol": "TM9SF3",
  "term_label": "membrane",
  "gene": "UniProtKB:Q9HD45",
  "term_id": "GO:0016020"
}